{
  "term_label": "Unknown molecular function",
  "gene_symbol": "CFAP119",
  "term_id": "UNKNOWN:0001",
  "gene_name": "Cilia- and flagella-associated protein 119",
  "gene": "UniProtKB:A1A4V9"
}